{
  "gene_name": "Liprin-alpha-1",
  "gene": "UniProtKB:Q13136",
  "term_id": "UNKNOWN:0001",
  "gene_symbol": "PPFIA1",
  "term_label": "Unknown molecular function"
}